circadian rhythm [GO:0007623] (BP) Definition: Any biological process in an organism that recurs with a regularity of approximately 24 hours. Relationships: is a type of GO:0048511 Subtypes: circadian regulation of systemic arterial blood pressure [GO:0003052], circadian regulation of heart rate [GO:0003053], circadian regulation of calcium ion oscillation [GO:0010617], circadian regulation of gene expression [GO:0032922], circadian behavior [GO:0048512], circadian temperature homeostasis [GO:0060086], circadian regulation of translation [GO:0097167] Also known as: circadian process, circadian response, response to circadian rhythm Sources: GOC:bf, GOC:go_curators Regulation: regulated by regulation of circadian rhythm [GO:0042752]; positively regulated by positive regulation of circadian rhythm [GO:0042753]; negatively regulated by GO:0042754